regulation of pancreatic juice secretion [GO:0090186] (biological process) Relationships: is a type of regulation of digestive system process [GO:0044058]; is a type of regulation of body fluid levels [GO:0050878]; is a type of regulation of secretion [GO:0051046]; regulates pancreatic juice secretion [GO:0030157] Subtypes: GO:0090187, negative regulation of pancreatic juice secretion [GO:0090188] Sources: GOC:dph, GOC:tb Definition: Any process that modulates the rate, frequency or extent of pancreatic juice secretion, the regulated release of pancreatic juice by the exocrine pancreas into the upper part of the intestine.